{
  "gene_name": "BPI fold-containing family B member 4",
  "gene": "UniProtKB:P59827",
  "term_id": "UNKNOWN:0002",
  "gene_symbol": "BPIFB4",
  "term_label": "Unknown biological process"
}